antisense RNA transcription [GO:0009300] (biological process) Definition: The synthesis of antisense RNA, an RNA molecule complementary in sequence to another RNA or DNA molecule, which, by binding the latter, acts to inhibit its function and/or completion of synthesis, on a template of DNA. Sources: GOC:jl Relationships: is a type of GO:0006351; is a type of GO:0042868 Regulation: regulated by regulation of antisense RNA transcription [GO:0060194]; negatively regulated by negative regulation of antisense RNA transcription [GO:0060195]; RO_0002213 by positive regulation of antisense RNA transcription [GO:0060196]